{
  "term_label": "cytosolic small ribosomal subunit",
  "term_id": "GO:0022627",
  "gene_symbol": "RPS3",
  "gene": "UniProtKB:P23396",
  "gene_name": "Small ribosomal subunit protein uS3"
}